calcium ion binding [GO:0005509] (molecular function) Definition: Binding to a calcium ion (Ca2+). Sources: GOC:ai Also known as: calcium ion storage activity Relationships: is a type of metal ion binding [GO:0046872] Subtypes: calcium ion binding involved in regulation of cytosolic calcium ion concentration [GO:0099510] Regulation: regulated by GO:1901876